C3HC4-type RING finger domain binding [GO:0055131] (molecular function) Relationships: is a type of protein domain specific binding [GO:0019904] Definition: Binding to a C3HC4-type zinc finger domain of a protein. The C3HC4-type zinc finger is a variant of RING finger, is a cysteine-rich domain of 40 to 60 residues that coordinates two zinc ions, and has the consensus sequence: C-X2-C-X(9-39)-C-X(1-3)-H-X(2-3)-C-X2-C-X(4-48)-C-X2-C, where X is any amino acid. Many proteins containing a C3HC4-type RING finger play a key role in the ubiquitination pathway. Sources: GOC:amm, InterPro:IPR001841, InterPro:IPR018957